{
  "gene_name": "D-beta-hydroxybutyrate dehydrogenase, mitochondrial",
  "gene": "UniProtKB:Q02338",
  "term_label": "Unknown cellular component",
  "gene_symbol": "BDH1",
  "term_id": "UNKNOWN:0003"
}